{
  "term_id": "GO:0007059",
  "term_label": "chromosome segregation",
  "gene_symbol": "SPC24",
  "gene_name": "Kinetochore protein Spc24",
  "gene": "UniProtKB:Q8NBT2"
}